{
  "gene": "UniProtKB:Q9C0B0",
  "term_label": "mRNA CDS binding",
  "term_id": "GO:1990715",
  "gene_name": "RING finger protein unkempt homolog",
  "gene_symbol": "UNK"
}